{
  "gene": "UniProtKB:A0A1W2PRN1",
  "term_id": "UNKNOWN:0003",
  "gene_name": "Golgin subfamily A conserved domain-containing protein",
  "term_label": "Unknown cellular component",
  "gene_symbol": "A0A1W2PRN1"
}